{
  "term_id": "GO:0005523",
  "gene_name": "Tropomodulin-4",
  "term_label": "tropomyosin binding",
  "gene_symbol": "TMOD4",
  "gene": "UniProtKB:Q9NZQ9"
}